alanopine dehydrogenase activity [GO:0047636] (molecular function) Also known as: 2,2'-iminodipropanoate:NAD+ oxidoreductase (L-alanine-forming), ADH, ALPDH, alanopine: NAD oxidoreductase activity, alanopine:NAD oxidoreductase activity, alanopine[meso-N-(1-carboxyethyl)-alanine]dehydrogenase activity, meso-N-(1-carboxyethyl)-alanine:NAD+ oxidoreductase activity Definition: Catalysis of the reaction: 2,2'-iminodipropanoate + H2O + NAD+ = L-alanine + H+ + NADH + pyruvate. Relationships: is a type of oxidoreductase activity, acting on the CH-NH group of donors, NAD or NADP as acceptor [GO:0016646] Sources: EC:1.5.1.17, RHEA:17589